{
  "term_id": "GO:0000209",
  "gene_symbol": "UBE3A",
  "term_label": "protein polyubiquitination",
  "gene": "UniProtKB:Q05086",
  "gene_name": "Ubiquitin-protein ligase E3A"
}